cellular response to erythromycin [GO:0072743] (biological process) Sources: GOC:mah Definition: Any process that results in a change in state or activity of a cell (in terms of movement, secretion, enzyme production, gene expression, etc.) as a result of an erythromycin stimulus. Relationships: is a type of response to erythromycin [GO:1901323]; is a type of cellular response to oxygen-containing compound [GO:1901701]